{
  "gene_name": "Glutamate-rich protein 3",
  "gene_symbol": "ERICH3",
  "term_label": "Unknown molecular function",
  "term_id": "UNKNOWN:0001",
  "gene": "UniProtKB:Q5RHP9"
}